autophagosome assembly [GO:0000045] (biological process) Regulation: negatively regulated by negative regulation of autophagosome assembly [GO:1902902]; regulated by regulation of autophagosome assembly [GO:2000785]; RO_0002213 by positive regulation of autophagosome assembly [GO:2000786] Definition: The formation of a double membrane-bounded structure, the autophagosome, that occurs when a specialized membrane sac, called the isolation membrane, starts to enclose a portion of the cytoplasm. References: PMID:9412464 Sources: GOC:autophagy Also known as: autophagic vacuole assembly, autophagosome biosynthesis, autophagosome formation, PAS formation, autophagic vacuole formation Relationships: is a type of organelle assembly [GO:0070925]; is a type of autophagosome organization [GO:1905037]; has part Atg12 activating enzyme activity [GO:0019778]; has part GO:0019786; has part GO:0061651; has part GO:0061660; has part Atg1/ULK1 kinase complex assembly [GO:1904745]